{
  "term_label": "Unknown molecular function",
  "gene_symbol": "LTO1",
  "gene_name": "Protein LTO1 homolog",
  "gene": "UniProtKB:Q8WV07",
  "term_id": "UNKNOWN:0001"
}